{
  "gene_symbol": "HELB",
  "gene_name": "DNA helicase B",
  "gene": "UniProtKB:Q8NG08",
  "term_id": "GO:0006974",
  "term_label": "DNA damage response"
}